marginal zone B cell differentiation [GO:0002315] (biological process) Definition: The process in which a B cell in the spleen acquires the specialized features of a marginal zone B cell. Marginal zone B cells are localized in a distinct anatomical region of the spleen that represents the major antigen-filtering and scavenging area (by specialized macrophages resident there). It appears that they are preselected to express a BCR repertoire similar to B-1 B cells, biased toward bacterial cell wall constituents and senescent self-components (such as oxidized LDL). Sources: GOC:jal, ISBN:0781735149 Relationships: is a type of mature B cell differentiation involved in immune response [GO:0002313] Note: Note that immunologists typically use the word 'development' to refer to cells of B or T cell lineages undergoing the process that GO describes as 'cell differentiation'. Also known as: marginal zone B lymphocyte differentiation, marginal zone B-cell differentiation, marginal zone B-lymphocyte differentiation, marginal zone B cell development